pyrenoid [GO:1990732] (cellular component) Definition: A non-membrane-bounded organelle found within the chloroplasts of algae and hornworts; responsible for carbon dioxide fixation. References: PMID:23345319 Sources: GOC:cjm, GOC:pr, Wikipedia:Pyrenoid Relationships: is a type of GO:0043232; is part of plastid [GO:0009536]